{
  "term_id": "UNKNOWN:0001",
  "gene": "UniProtKB:Q8NBI3",
  "gene_symbol": "DRAXIN",
  "term_label": "Unknown molecular function",
  "gene_name": "Draxin"
}